regulation of forebrain neuron differentiation [GO:2000977] (biological process) Definition: Any process that modulates the frequency, rate or extent of forebrain neuron differentiation. Sources: GOC:obol Relationships: is a type of regulation of neuron differentiation [GO:0045664]; regulates GO:0021879 Subtypes: negative regulation of forebrain neuron differentiation [GO:2000978], positive regulation of forebrain neuron differentiation [GO:2000979]